{
  "term_label": "positive regulation of cytokinesis",
  "term_id": "GO:0032467",
  "gene_symbol": "CDC14B",
  "gene": "UniProtKB:O60729",
  "gene_name": "Dual specificity protein phosphatase CDC14B"
}